{
  "gene_name": "Humanin-like 3",
  "term_id": "GO:1900118",
  "term_label": "negative regulation of execution phase of apoptosis",
  "gene_symbol": "MTRNR2L3",
  "gene": "UniProtKB:P0CJ70"
}